{
  "gene_symbol": "BIK",
  "term_label": "Unknown molecular function",
  "gene": "UniProtKB:Q13323",
  "gene_name": "Bcl-2-interacting killer",
  "term_id": "UNKNOWN:0001"
}